{
  "gene_name": "Putative uncharacterized protein SCP2D1-AS1",
  "gene_symbol": "SCP2D1-AS1",
  "gene": "UniProtKB:Q9BR46",
  "term_id": "UNKNOWN:0001",
  "term_label": "Unknown molecular function"
}